{
  "term_id": "GO:0071280",
  "gene_symbol": "MT1HL1",
  "term_label": "cellular response to copper ion",
  "gene_name": "Metallothionein 1H-like protein 1",
  "gene": "UniProtKB:P0DM35"
}